{
  "gene": "UniProtKB:Q86W74",
  "term_label": "Unknown cellular component",
  "term_id": "UNKNOWN:0003",
  "gene_name": "Ankyrin repeat domain-containing protein 46",
  "gene_symbol": "ANKRD46"
}